{
  "term_label": "Prp19 complex",
  "gene": "UniProtKB:Q99459",
  "term_id": "GO:0000974",
  "gene_name": "Cell division cycle 5-like protein",
  "gene_symbol": "CDC5L"
}